{
  "gene_symbol": "ROCK1",
  "term_label": "cytoskeleton",
  "gene": "UniProtKB:Q13464",
  "gene_name": "Rho-associated protein kinase 1",
  "term_id": "GO:0005856"
}